{
  "term_id": "GO:0051058",
  "gene_symbol": "ARHGAP25",
  "gene_name": "Rho GTPase-activating protein 25",
  "term_label": "negative regulation of small GTPase mediated signal transduction",
  "gene": "UniProtKB:P42331"
}